dGDP catabolic process [GO:0046067] (biological process) Definition: The chemical reactions and pathways resulting in the breakdown of dGDP, deoxyguanosine diphosphate, (2'-deoxyguanosine 5'-diphosphate). Also known as: dGDP breakdown, dGDP catabolism, dGDP degradation Sources: GOC:go_curators Relationships: is a type of purine deoxyribonucleotide catabolic process [GO:0009155]; is a type of GO:0009184; is a type of dGDP metabolic process [GO:0046066]